{
  "term_id": "GO:0030490",
  "gene_symbol": "NOP14",
  "gene_name": "Nucleolar protein 14",
  "term_label": "maturation of SSU-rRNA",
  "gene": "UniProtKB:P78316"
}